{
  "gene_symbol": "HSD17B14",
  "term_label": "Unknown molecular function",
  "term_id": "UNKNOWN:0001",
  "gene": "UniProtKB:Q9BPX1",
  "gene_name": "17-beta-hydroxysteroid dehydrogenase 14"
}